{
  "gene_symbol": "ZNF669",
  "term_id": "GO:0005634",
  "gene_name": "Zinc finger protein 669",
  "gene": "UniProtKB:Q96BR6",
  "term_label": "nucleus"
}